{
  "gene": "UniProtKB:Q02447",
  "gene_symbol": "SP3",
  "gene_name": "Transcription factor Sp3",
  "term_id": "GO:0000978",
  "term_label": "RNA polymerase II cis-regulatory region sequence-specific DNA binding"
}